{
  "gene_symbol": "GAMT",
  "term_id": "GO:0030731",
  "term_label": "guanidinoacetate N-methyltransferase activity",
  "gene_name": "Guanidinoacetate N-methyltransferase",
  "gene": "UniProtKB:Q14353"
}